positive regulation of cytosolic calcium ion concentration [GO:0007204] (BP) Subtypes: positive regulation of calcium ion transport into cytosol [GO:0010524], calcium ion transport into cytosol [GO:0060402], positive regulation of cytosolic calcium ion concentration involved in egg activation [GO:0060470], GO:0099533, GO:0099588 Also known as: cytoplasmic calcium ion concentration elevation, elevation of calcium ion concentration in cytoplasm, elevation of cytoplasmic calcium ion concentration, cytosolic calcium ion concentration elevation, elevation of calcium ion concentration in cytosol, elevation of cytosolic calcium ion concentration Relationships: is a type of regulation of biological quality [GO:0065008] Sources: GOC:ai Definition: Any process that increases the concentration of calcium ions in the cytosol.